{
  "term_id": "GO:0005634",
  "gene_symbol": "ZNF93",
  "term_label": "nucleus",
  "gene": "UniProtKB:P35789",
  "gene_name": "Zinc finger protein 93"
}